galacturonan metabolic process [GO:0010393] (biological process) Subtypes: homogalacturonan metabolic process [GO:0010394], xylogalacturonan metabolic process [GO:0010398], pectin metabolic process [GO:0045488] Sources: GOC:tair_curators Definition: The chemical reactions and pathways involving galacturonan, a pectin polymer containing a backbone of alpha-(1->4)-linked D-galacturonic acid residues. Also known as: galacturonan metabolism Relationships: is a type of GO:0005976